filopodium membrane [GO:0031527] (cellular component) Definition: The portion of the plasma membrane surrounding a filopodium. Sources: GOC:mah Relationships: is a type of cell projection membrane [GO:0031253]; BFO_0000050 GO:0030175